transnitrosylase complex [GO:1990658] (cellular component) Subtypes: iNOS-S100A8/A9 complex [GO:1990657] References: PMID:25417112 Sources: GOC:bhm Relationships: is a type of transferase complex [GO:1990234]; is part of GO:0005737 Also known as: transferase complex, transferring nitrogenous groups Definition: A transferase complex which is capable of transferring nitrogenous groups from one component to another. Note: An example of this is S100A9 in human (UniProt symbol P06702) in PMID:25417112 (inferred from direct assay).